{
  "gene_symbol": "OR10H3",
  "gene": "UniProtKB:O60404",
  "term_id": "GO:0050911",
  "term_label": "detection of chemical stimulus involved in sensory perception of smell",
  "gene_name": "Olfactory receptor 10H3"
}